{
  "term_id": "GO:0000122",
  "gene": "UniProtKB:Q6NUN9",
  "term_label": "negative regulation of transcription by RNA polymerase II",
  "gene_symbol": "ZNF746",
  "gene_name": "Zinc finger protein 746"
}